{
  "gene": "UniProtKB:Q6ZR62",
  "gene_symbol": "RTL4",
  "term_label": "Unknown cellular component",
  "term_id": "UNKNOWN:0003",
  "gene_name": "Retrotransposon Gag-like protein 4"
}